clathrin adaptor activity [GO:0035615] (molecular function) References: PMID:15728179 Sources: GOC:BHF Definition: Bringing together a cargo protein with clathrin, responsible for the formation of endocytic vesicles. Relationships: is a type of cargo adaptor activity [GO:0140312]; has part clathrin binding [GO:0030276] Also known as: clathrin-associated adaptor activity